{
  "gene_symbol": "FCN1",
  "term_id": "GO:0003823",
  "gene_name": "Ficolin-1",
  "term_label": "antigen binding",
  "gene": "UniProtKB:O00602"
}